positive regulation of neurotrophin production [GO:0032901] (biological process) Also known as: up regulation of neurotrophin production, up-regulation of neurotrophin production, upregulation of neurotrophin production, activation of neurotrophin production, stimulation of neurotrophin production Definition: Any process that activates or increases the frequency, rate, or extent of production of a neurotrophin. Relationships: is a type of regulation of neurotrophin production [GO:0032899]; is a type of positive regulation of multicellular organismal process [GO:0051240]; positively regulates neurotrophin production [GO:0032898] Sources: GOC:mah